{
  "gene_name": "Doublesex- and mab-3-related transcription factor C2",
  "term_label": "Unknown biological process",
  "gene": "UniProtKB:Q8IXT2",
  "gene_symbol": "DMRTC2",
  "term_id": "UNKNOWN:0002"
}